{
  "gene_name": "Bone morphogenetic protein receptor type-1A",
  "gene": "UniProtKB:P36894",
  "term_id": "GO:0005025",
  "gene_symbol": "BMPR1A",
  "term_label": "transforming growth factor beta receptor activity, type I"
}